{
  "term_id": "GO:0045494",
  "term_label": "photoreceptor cell maintenance",
  "gene": "UniProtKB:Q8IWN7",
  "gene_symbol": "RP1L1",
  "gene_name": "Retinitis pigmentosa 1-like 1 protein"
}